{
  "term_label": "'de novo' cotranslational protein folding",
  "gene": "UniProtKB:Q9Y4R8",
  "gene_symbol": "TELO2",
  "term_id": "GO:0051083",
  "gene_name": "Telomere length regulation protein TEL2 homolog"
}